{
  "gene_name": "Mitochondrial glutamate carrier 1",
  "gene": "UniProtKB:Q9H936",
  "gene_symbol": "SLC25A22",
  "term_label": "malate-aspartate shuttle",
  "term_id": "GO:0043490"
}